{
  "gene": "UniProtKB:Q9NX76",
  "term_id": "UNKNOWN:0001",
  "gene_name": "CKLF-like MARVEL transmembrane domain-containing protein 6",
  "term_label": "Unknown molecular function",
  "gene_symbol": "CMTM6"
}